{
  "gene_name": "Protein NKG7",
  "term_label": "plasma membrane",
  "gene_symbol": "NKG7",
  "gene": "UniProtKB:Q16617",
  "term_id": "GO:0005886"
}